{
  "gene_name": "Bridge-like lipid transfer protein family member 2",
  "term_label": "Unknown cellular component",
  "gene_symbol": "BLTP2",
  "term_id": "UNKNOWN:0003",
  "gene": "UniProtKB:Q14667"
}